B-WICH complex [GO:0110016] (cellular component) Relationships: is a type of SWI/SNF superfamily-type complex [GO:0070603]; is part of nucleolus [GO:0005730] Note: An example is BAZ1B (Q9UIG0) in human in PMID:16603771 (by IPI). References: PMID:16603771, PMID:21559432, PMID:23555303, PMID:26044184 Sources: GOC:bhm Definition: A chromatin remodeling complex that positively regulates histone H3 acetylation, in particular H3K9, by recruiting histone acetyltransferases to rDNA gene regions. Located in the nucleolus where it assembles on RNA Polymerase I (Pol I) and possibly on RNA Polymerase III (Pol III) promoter and coding regions during early G1 phase and activates the post-initiation phases of Pol I transcription. May also activate RNA Polymerase II (Pol II) gene transcription. In mammals, B-WICH contains the WICH complex core of BAZ1B and SMARCA5, additional protein subunits and possibly rRNAs. Although it contains several catalytic subunits it is not clear which functions are carried out by the complex itself.